{
  "gene": "UniProtKB:P17538",
  "gene_name": "Chymotrypsinogen B",
  "term_label": "Unknown cellular component",
  "gene_symbol": "CTRB1",
  "term_id": "UNKNOWN:0003"
}